{
  "term_label": "regulated exocytosis",
  "gene_name": "Rab11 family-interacting protein 2",
  "gene_symbol": "RAB11FIP2",
  "gene": "UniProtKB:Q7L804",
  "term_id": "GO:0045055"
}